{
  "gene_symbol": "CENPK",
  "term_label": "mitotic sister chromatid segregation",
  "gene_name": "Centromere protein K",
  "term_id": "GO:0000070",
  "gene": "UniProtKB:Q9BS16"
}